phytochelatin import into vacuole [GO:0071995] (biological process) Definition: The directed movement of phytochelatins into the vacuole. Phytochelatins are a group of peptides that bind metals (Cd, Zn, Cu, Pb, Hg) in thiolate coordination complexes. Sources: GOC:mah, ISBN:0198506732 Also known as: phytochelatin transport into vacuole, cadystin import into vacuole Relationships: is a type of vacuolar transmembrane transport [GO:0034486]; is_a phytochelatin transmembrane transport [GO:0071994] Subtypes: GO:0036246, phytochelatin 3 import into vacuole [GO:0036247], GO:0036248